{
  "gene": "UniProtKB:Q969T7",
  "gene_name": "7-methylguanosine phosphate-specific 5'-nucleotidase",
  "term_id": "GO:0005737",
  "gene_symbol": "NT5C3B",
  "term_label": "cytoplasm"
}